{
  "gene_symbol": "CENPC",
  "gene": "UniProtKB:Q03188",
  "term_id": "GO:0051315",
  "term_label": "attachment of mitotic spindle microtubules to kinetochore",
  "gene_name": "Centromere protein C"
}